{
  "gene_name": "Cytoplasmic dynein 1 heavy chain 1",
  "gene_symbol": "DYNC1H1",
  "term_id": "GO:0045505",
  "gene": "UniProtKB:Q14204",
  "term_label": "dynein intermediate chain binding"
}